{
  "gene_symbol": "LAYN",
  "term_label": "Unknown cellular component",
  "gene_name": "Layilin",
  "term_id": "UNKNOWN:0003",
  "gene": "UniProtKB:Q6UX15"
}